{
  "term_id": "UNKNOWN:0002",
  "gene_symbol": "MRPL48",
  "term_label": "Unknown biological process",
  "gene": "UniProtKB:Q96GC5",
  "gene_name": "Large ribosomal subunit protein mL48"
}